{
  "term_label": "negative regulation of smoothened signaling pathway",
  "term_id": "GO:0045879",
  "gene_symbol": "MOSMO",
  "gene_name": "Modulator of smoothened protein",
  "gene": "UniProtKB:Q8NHV5"
}